{
  "gene_name": "Serine_threonine-protein kinase mTOR",
  "gene": "UniProtKB:P42345",
  "term_id": "GO:0005634",
  "gene_symbol": "MTOR",
  "term_label": "nucleus"
}